cellular response to interleukin-32 [GO:0097397] (biological process) Sources: GOC:pr Relationships: is a type of cellular response to cytokine stimulus [GO:0071345]; is a type of GO:0097395 Also known as: cellular response to IL-32 Definition: Any process that results in a change in state or activity of a cell (in terms of movement, secretion, enzyme production, gene expression, etc.) as a result of an interleukin-32 stimulus.